beta-glucoside biosynthetic process [GO:1901806] (biological process) Definition: The chemical reactions and pathways resulting in the formation of beta-glucoside. Subtypes: dhurrin biosynthetic process [GO:0010132], kaempferol O-glucoside biosynthetic process [GO:0033330], cyanidin 3-O-glucoside biosynthetic process [GO:0033485], delphinidin 3-O-glucoside biosynthetic process [GO:0033486], pelargonidin 3-O-glucoside biosynthetic process [GO:0033487], (-)-secologanin biosynthetic process [GO:1900994], 3alpha(S)-strictosidine biosynthetic process [GO:1901015], zeaxanthin bis(beta-D-glucoside) biosynthetic process [GO:1901830], ergosteryl 3-beta-D-glucoside biosynthetic process [GO:1904463] Relationships: is a type of glycoside biosynthetic process [GO:0016138] References: PMID:15205427, PMID:16390337, PMID:8990303 Sources: GOC:TermGenie, GOC:yaf, Unipathway:UPA00237 Also known as: beta-glucoside anabolism, beta-glucoside biosynthesis, beta-glucoside formation, beta-glucoside synthesis